{
  "gene_symbol": "MRPL57",
  "gene_name": "Large ribosomal subunit protein mL63",
  "term_label": "Unknown biological process",
  "gene": "UniProtKB:Q9BQC6",
  "term_id": "UNKNOWN:0002"
}